{
  "term_label": "negative regulation of complement activation, classical pathway",
  "term_id": "GO:0045959",
  "gene_name": "C4b-binding protein alpha chain",
  "gene": "UniProtKB:P04003",
  "gene_symbol": "C4BPA"
}